{
  "term_label": "Unknown molecular function",
  "gene_symbol": "IGKV2D-26",
  "gene": "UniProtKB:A0A0A0MRZ7",
  "term_id": "UNKNOWN:0001",
  "gene_name": "Immunoglobulin kappa variable 2D-26"
}